{
  "gene": "UniProtKB:Q8WUH1",
  "gene_name": "Protein Churchill",
  "gene_symbol": "CHURC1",
  "term_label": "Unknown molecular function",
  "term_id": "UNKNOWN:0001"
}